exit of virus from host cell nucleus through nuclear pore [GO:0039675] (biological process) Definition: The directed movement of the viral genome or a viral particle out of the host cell nucleus through the nuclear pore. Also known as: exit of virus from host cell nucleus through nuclear pore complex, nuclear pore exit of virus, viral enome export through nuclear pore Relationships: is a type of exit of virus from host cell nucleus [GO:0039674] References: PMID:12921991 Sources: VZ:1953